{
  "gene_name": "Protocadherin gamma-A1",
  "gene": "UniProtKB:Q9Y5H4",
  "term_id": "GO:0050839",
  "term_label": "cell adhesion molecule binding",
  "gene_symbol": "PCDHGA1"
}